{
  "term_id": "GO:0001530",
  "term_label": "lipopolysaccharide binding",
  "gene": "UniProtKB:Q96DR5",
  "gene_symbol": "BPIFA2",
  "gene_name": "BPI fold-containing family A member 2"
}